{
  "gene": "UniProtKB:P61758",
  "term_id": "GO:0007017",
  "gene_symbol": "VBP1",
  "gene_name": "Prefoldin subunit 3",
  "term_label": "microtubule-based process"
}